galactoside binding [GO:0016936] (MF) Definition: Binding to a glycoside in which the sugar group is galactose. Relationships: is_a carbohydrate derivative binding [GO:0097367] Sources: GOC:jl, ISBN:0198506732